{
  "gene": "UniProtKB:Q8IZT9",
  "term_label": "synaptonemal complex",
  "gene_symbol": "FAM9C",
  "gene_name": "Protein FAM9C",
  "term_id": "GO:0000795"
}